{
  "gene_symbol": "LCP2",
  "gene": "UniProtKB:Q13094",
  "term_label": "intracellular signal transduction",
  "term_id": "GO:0035556",
  "gene_name": "Lymphocyte cytosolic protein 2"
}